regulation of MDA-5 signaling pathway [GO:0039533] (biological process) Definition: Any process that modulates the frequency, rate or extent of the series of molecular signals generated as a consequence of the cytoplasmic pattern recognition receptor (PRR) MDA-5 (also known as IFIH1) binding to viral RNA. Also known as: regulation of IFIH1 signaling pathway, regulation of MDA-5 signalling pathway, regulation of MDA5 signaling pathway, regulation of melanoma differentiation-associated gene 5 signaling pathway Relationships: is a type of regulation of cytoplasmic pattern recognition receptor signaling pathway [GO:0039531]; regulates MDA-5 signaling pathway [GO:0039530] Sources: GOC:bf, GOC:jl Subtypes: negative regulation of MDA-5 signaling pathway [GO:0039534], GO:1900245